{
  "gene_name": "Nibrin",
  "term_id": "GO:0000724",
  "gene": "UniProtKB:O60934",
  "term_label": "double-strand break repair via homologous recombination",
  "gene_symbol": "NBN"
}